protein transport to vacuole involved in ubiquitin-dependent protein catabolic process via the multivesicular body sorting pathway [GO:0043328] (biological process) References: PMID:11511343 Sources: GOC:jl Relationships: is a type of intracellular protein transport [GO:0006886]; is a type of GO:0032511; is a type of protein localization to vacuole [GO:0072665]; is a type of GO:0072666; is part of ubiquitin-dependent protein catabolic process via the multivesicular body sorting pathway [GO:0043162] Also known as: protein targeting to vacuole during ubiquitin-dependent protein breakdown via the MVB pathway, protein targeting to vacuole during ubiquitin-dependent protein degradation via the MVB pathway, protein vacuolar targeting during ubiquitin-dependent protein catabolic process via the MVB pathway, protein vacuolar targeting during ubiquitin-dependent protein catabolism via the MVB pathway, protein-vacuolar targeting during ubiquitin-dependent protein breakdown via the MVB pathway, protein-vacuolar targeting during ubiquitin-dependent protein degradation via the MVB pathway, protein-vacuole targeting during ubiquitin-dependent protein catabolic process via the MVB pathway, protein-vacuole targeting during ubiquitin-dependent protein catabolism via the MVB pathway, protein targeting to vacuole during ubiquitin-dependent protein catabolic process via the MVB pathway Definition: The process of directing proteins towards the vacuole that contributes to protein catabolism via the multivesicular body (MVB) pathway.